rhombomere 5 morphogenesis [GO:0021664] (biological process) Definition: The process in which the anatomical structures of rhombomere 5 are generated and organized. Rhombomeres are transverse segments of the developing rhombencephalon. Rhombomeres are lineage restricted, express different genes from one another, and adopt different developmental fates. Rhombomeres are numbered in an anterior to posterior order. Sources: GOC:cls, GOC:dgh, GOC:dph, GOC:jid, GO_REF:0000021 Relationships: is a type of rhombomere morphogenesis [GO:0021593]; is part of rhombomere 5 development [GO:0021571]